hexose uniporter activity [GO:0008516] (molecular function) Relationships: is a type of GO:0015149; is_a uniporter activity [GO:0015292] Definition: Enables the transfer of a solute or solutes from one side of a membrane to the other according to the reaction: hexose(out) = hexose(in). Subtypes: fructose uniporter activity [GO:0015284], D-glucose uniporter activity [GO:0015304], galactose uniporter activity [GO:0050782] Sources: TC:2.A.1.1.5